{
  "gene_name": "CKLF-like MARVEL transmembrane domain-containing protein 1",
  "gene_symbol": "CMTM1",
  "term_label": "Unknown molecular function",
  "gene": "UniProtKB:Q8IZ96",
  "term_id": "UNKNOWN:0001"
}